{
  "gene_name": "Tetratricopeptide repeat protein 14",
  "term_label": "Unknown cellular component",
  "term_id": "UNKNOWN:0003",
  "gene": "UniProtKB:Q96N46",
  "gene_symbol": "TTC14"
}